{
  "term_id": "GO:0043005",
  "gene": "UniProtKB:P41145",
  "gene_symbol": "OPRK1",
  "gene_name": "Kappa-type opioid receptor",
  "term_label": "neuron projection"
}